{
  "term_id": "GO:0016538",
  "gene_symbol": "CCNE2",
  "term_label": "cyclin-dependent protein serine/threonine kinase regulator activity",
  "gene": "UniProtKB:O96020",
  "gene_name": "G1_S-specific cyclin-E2"
}